{
  "gene_name": "Protein Wnt-8b",
  "gene": "UniProtKB:Q93098",
  "term_label": "frizzled binding",
  "gene_symbol": "WNT8B",
  "term_id": "GO:0005109"
}